{
  "term_label": "Unknown molecular function",
  "gene_symbol": "SPINK2",
  "gene_name": "Serine protease inhibitor Kazal-type 2",
  "term_id": "UNKNOWN:0001",
  "gene": "UniProtKB:P20155"
}